(-)-microperfuranone biosynthetic process [GO:1901512] (biological process) Relationships: is a type of lactone biosynthetic process [GO:1901336]; is_a ether biosynthetic process [GO:1901503] Sources: GOC:TermGenie, GOC:di Also known as: (-)-microperfuranone anabolism, (-)-microperfuranone biosynthesis, (-)-microperfuranone formation, (-)-microperfuranone synthesis Definition: The chemical reactions and pathways resulting in the formation of (-)-microperfuranone.